{
  "term_id": "GO:0006511",
  "gene_name": "Ubiquitin D",
  "gene": "UniProtKB:O15205",
  "term_label": "ubiquitin-dependent protein catabolic process",
  "gene_symbol": "UBD"
}